{
  "gene_symbol": "OR1L1",
  "term_id": "GO:0004984",
  "gene_name": "Olfactory receptor 1L1",
  "term_label": "olfactory receptor activity",
  "gene": "UniProtKB:Q8NH94"
}